cellular response to methylmercury [GO:0071406] (biological process) Sources: GOC:mah Relationships: is a type of GO:0051597 Also known as: cellular response to CH3-Hg+, cellular response to MeHg+ Definition: Any process that results in a change in state or activity of a cell (in terms of movement, secretion, enzyme production, gene expression, etc.) as a result of a methylmercury stimulus.